{
  "gene_symbol": "HNRNPCL3",
  "gene_name": "Heterogeneous nuclear ribonucleoprotein C-like 3",
  "gene": "UniProtKB:B7ZW38",
  "term_label": "nucleus",
  "term_id": "GO:0005634"
}